{
  "gene_symbol": "ELP1",
  "term_id": "GO:0002926",
  "gene_name": "Elongator complex protein 1",
  "term_label": "tRNA wobble base 5-methoxycarbonylmethyl-2-thiouridinylation",
  "gene": "UniProtKB:O95163"
}